inner nuclear membrane-associated protein degradation pathway [GO:0180027] (biological process) Also known as: INMAD pathway Definition: A protein quality control pathway that removes ubiquitinated proteins from the nuclear inner membrane before transferring them to the proteasome for degradation. Relationships: is a type of nuclear protein quality control by the ubiquitin-proteasome system [GO:0071630] References: PMID:37694715